{
  "gene_name": "H(+)_Cl(-) exchange transporter 7",
  "term_id": "GO:0030321",
  "gene_symbol": "CLCN7",
  "gene": "UniProtKB:P51798",
  "term_label": "transepithelial chloride transport"
}